{
  "term_id": "GO:0005737",
  "gene_symbol": "MOK",
  "gene_name": "MAPK_MAK_MRK overlapping kinase",
  "gene": "UniProtKB:Q9UQ07",
  "term_label": "cytoplasm"
}